cardiac chamber development [GO:0003205] (biological process) Relationships: is a type of anatomical structure development [GO:0048856]; is part of GO:0007507 Definition: The progression of a cardiac chamber over time, from its formation to the mature structure. A cardiac chamber is an enclosed cavity within the heart. Sources: GOC:mtg_heart Subtypes: cardiac atrium development [GO:0003230], cardiac ventricle development [GO:0003231], bulbus arteriosus development [GO:0003232], sinus venosus development [GO:0003235], conus arteriosus development [GO:0003238]